neural crest-derived cardiac fibroblast cell development [GO:0060943] (biological process) Sources: GOC:mtg_heart Relationships: is a type of GO:0060936; is part of GO:0060942 Definition: The process whose specific outcome is the progression of a cardiac fibroblast over time, from its formation from a neural crest cell to the mature state. A cardiac fibroblast is a connective tissue cell of the heart which secretes an extracellular matrix rich in collagen and other macromolecules.